{
  "gene_symbol": "ATP6V1B1",
  "gene_name": "V-type proton ATPase subunit B, kidney isoform",
  "gene": "UniProtKB:P15313",
  "term_label": "plasma membrane",
  "term_id": "GO:0005886"
}